{
  "gene_symbol": "LSM7",
  "gene_name": "U6 snRNA-associated Sm-like protein LSm7",
  "gene": "UniProtKB:Q9UK45",
  "term_id": "GO:0005688",
  "term_label": "U6 snRNP"
}